{
  "gene_name": "Phosphoserine aminotransferase",
  "gene_symbol": "PSAT1",
  "gene": "UniProtKB:Q9Y617",
  "term_label": "L-serine biosynthetic process",
  "term_id": "GO:0006564"
}